{
  "term_id": "GO:0008017",
  "term_label": "microtubule binding",
  "gene": "UniProtKB:O43663",
  "gene_symbol": "PRC1",
  "gene_name": "Protein regulator of cytokinesis 1"
}